{
  "gene_symbol": "ZNF280C",
  "term_label": "Unknown cellular component",
  "term_id": "UNKNOWN:0003",
  "gene": "UniProtKB:Q8ND82",
  "gene_name": "Zinc finger protein 280C"
}